{
  "term_label": "positive regulation of cell population proliferation",
  "gene": "UniProtKB:Q8IZC4",
  "gene_name": "Rhotekin-2",
  "gene_symbol": "RTKN2",
  "term_id": "GO:0008284"
}